{
  "gene_name": "Forkhead box protein J3",
  "term_label": "RNA polymerase II cis-regulatory region sequence-specific DNA binding",
  "gene": "UniProtKB:Q9UPW0",
  "term_id": "GO:0000978",
  "gene_symbol": "FOXJ3"
}